polyprenol reductase activity [GO:0102389] (MF) Relationships: is_a oxidoreductase activity, acting on the CH-CH group of donors, NAD or NADP as acceptor [GO:0016628] Sources: GOC:pz, RHEA:34279 Definition: Catalysis of the reaction: NADP + a ditrans,polycis-dolichol = NADPH + H+ + a di-trans, poly-cis-polyprenol.